{
  "term_label": "platelet activation",
  "gene_symbol": "TREML1",
  "term_id": "GO:0030168",
  "gene_name": "Trem-like transcript 1 protein",
  "gene": "UniProtKB:Q86YW5"
}